phagosome-lysosome docking involved in apoptotic cell clearance [GO:0090388] (biological process) Definition: The initial attachment of a phagosome membrane to a lysosome membrane that occurs as a part of apoptotic cell clearance. Docking requires only that the proteins come close enough to interact and adhere. Sources: GOC:kmv, GOC:tb Relationships: is a type of phagosome-lysosome docking [GO:0090384]; is part of phagolysosome assembly involved in apoptotic cell clearance [GO:0090387]